{
  "gene": "UniProtKB:Q86UA6",
  "gene_name": "RPA-interacting protein",
  "term_id": "GO:0006606",
  "term_label": "protein import into nucleus",
  "gene_symbol": "RPAIN"
}